sepal development [GO:0048442] (BP) Relationships: is a type of floral organ development [GO:0048437]; is a type of GO:0048827; is part of flower calyx development [GO:0048464] Definition: The process whose specific outcome is the progression of the sepal over time, from its formation to the mature structure. Sources: GOC:go_curators